{
  "gene_symbol": "CD9",
  "term_id": "UNKNOWN:0001",
  "term_label": "Unknown molecular function",
  "gene_name": "CD9 antigen",
  "gene": "UniProtKB:P21926"
}